{
  "gene_name": "Diphosphoinositol polyphosphate phosphohydrolase NUDT4B",
  "gene_symbol": "NUDT4B",
  "gene": "UniProtKB:A0A024RBG1",
  "term_id": "GO:1901907",
  "term_label": "diadenosine pentaphosphate catabolic process"
}